{
  "term_label": "determination of left/right symmetry",
  "gene_symbol": "CFC1",
  "term_id": "GO:0007368",
  "gene": "UniProtKB:P0CG37",
  "gene_name": "Cryptic protein"
}